octopamine catabolic process [GO:0046334] (biological process) Definition: The chemical reactions and pathways resulting in the breakdown of octopamine, 1-(p-hydroxyphenyl)-2-aminoethanol. The D enantiomer is about one-tenth as active as norepinephrine and is found in the salivary glands of Octopus and Eledone species. Sources: ISBN:0198506732 Also known as: octopamine breakdown, octopamine catabolism, octopamine degradation Relationships: is a type of phenol-containing compound catabolic process [GO:0019336]; is a type of biogenic amine catabolic process [GO:0042402]; is_a alcohol catabolic process [GO:0046164]; is a type of octopamine metabolic process [GO:0046333]